lysosomal multienzyme complex [GO:0070559] (cellular component) Also known as: GALNS-lysosomal hydrolase 1.27 MDa complex Relationships: is a type of catalytic complex [GO:1902494]; is part of lysosome [GO:0005764] Definition: A protein complex found in the lysosome that contains beta-galactosidase, cathepsin A, alpha-neuraminidase and N-acetylgalactosamine-6-sulfate sulfatase, and is involved in glycosaminoglycan catabolism. References: PMID:8910459 Sources: GOC:mah